positive regulation of tensidol A biosynthetic process [GO:1900709] (biological process) Also known as: activation of tensidol A anabolism, activation of tensidol A biosynthesis, activation of tensidol A formation, activation of tensidol A synthesis, positive regulation of tensidol A anabolism, positive regulation of tensidol A biosynthesis, positive regulation of tensidol A formation, positive regulation of tensidol A synthesis, up regulation of tensidol A anabolism, up regulation of tensidol A biosynthesis, up regulation of tensidol A biosynthetic process, up regulation of tensidol A formation, up regulation of tensidol A synthesis, up-regulation of tensidol A anabolism, up-regulation of tensidol A biosynthesis, up-regulation of tensidol A biosynthetic process, up-regulation of tensidol A formation, up-regulation of tensidol A synthesis, upregulation of tensidol A anabolism, upregulation of tensidol A biosynthesis, upregulation of tensidol A biosynthetic process, upregulation of tensidol A formation, upregulation of tensidol A synthesis, activation of tensidol A biosynthetic process Relationships: is a type of positive regulation of amide metabolic process [GO:0034250]; is a type of GO:0062013; is a type of positive regulation of secondary metabolite biosynthetic process [GO:1900378]; is a type of regulation of tensidol A biosynthetic process [GO:1900707]; positively regulates tensidol A biosynthetic process [GO:1900605] Definition: Any process that activates or increases the frequency, rate or extent of tensidol A biosynthetic process. Sources: GOC:TermGenie, GOC:di